{
  "gene_name": "Proton-coupled zinc antiporter SLC30A1",
  "gene": "UniProtKB:Q9Y6M5",
  "term_id": "GO:0006882",
  "term_label": "intracellular zinc ion homeostasis",
  "gene_symbol": "SLC30A1"
}